DNA-(abasic site) binding [GO:0140431] (molecular function) Also known as: DNA AP site binding, DNA-(apurinic site/apyrimidinic site) binding, DNA-(apurinic site) binding, DNA-(apyrimidinic site) binding References: PMID:23245849 Definition: Binding to a DNA site that has neither a purine nor a pyrimidine base. Apurinic sites can form spontaneously or when DNA glycosylase removes a damaged base. Relationships: is a type of damaged DNA binding [GO:0003684]